{
  "gene_name": "Protein FAM186A",
  "gene": "UniProtKB:A6NE01",
  "term_id": "UNKNOWN:0002",
  "term_label": "Unknown biological process",
  "gene_symbol": "FAM186A"
}